negative regulation of glycogen (starch) synthase activity [GO:2000466] (biological process) Also known as: negative regulation of UDP-glucose-glycogen glucosyltransferase activity, negative regulation of UDP-glucose:glycogen 4-alpha-D-glucosyltransferase activity, negative regulation of UDP-glycogen synthase activity, negative regulation of UDPG-glycogen synthetase activity, negative regulation of UDPG-glycogen transglucosylase activity, negative regulation of UDPglucose:glycogen 4-alpha-D-glucosyltransferase activity, negative regulation of glycogen (starch) synthetase activity, negative regulation of uridine diphosphoglucose-glycogen glucosyltransferase activity Sources: GOC:obol Definition: Any process that stops, prevents or reduces the frequency, rate or extent of glycogen (starch) synthase activity. Relationships: is a type of negative regulation of catalytic activity [GO:0043086]; is a type of regulation of glycogen (starch) synthase activity [GO:2000465]; negatively regulates alpha-1,4-glucan glucosyltransferase (UDP-glucose donor) activity [GO:0004373]